{
  "gene_name": "Protocadherin beta-2",
  "term_id": "GO:0005886",
  "gene_symbol": "PCDHB2",
  "term_label": "plasma membrane",
  "gene": "UniProtKB:Q9Y5E7"
}